{
  "gene": "UniProtKB:P05230",
  "gene_symbol": "FGF1",
  "term_id": "GO:0022008",
  "gene_name": "Fibroblast growth factor 1",
  "term_label": "neurogenesis"
}